positive regulation of antigen processing and presentation of polysaccharide antigen via MHC class II [GO:0002603] (biological process) Sources: GOC:add Also known as: positive regulation of polysaccharide antigen processing and presentation via MHC class II, up regulation of antigen processing and presentation of polysaccharide antigen via MHC class II, up-regulation of antigen processing and presentation of polysaccharide antigen via MHC class II, upregulation of antigen processing and presentation of polysaccharide antigen via MHC class II, activation of antigen processing and presentation of polysaccharide antigen via MHC class II, stimulation of antigen processing and presentation of polysaccharide antigen via MHC class II Relationships: is a type of positive regulation of antigen processing and presentation of peptide or polysaccharide antigen via MHC class II [GO:0002582]; is a type of regulation of antigen processing and presentation of polysaccharide antigen via MHC class II [GO:0002601]; positively regulates antigen processing and presentation of polysaccharide antigen via MHC class II [GO:0002505] Definition: Any process that activates or increases the frequency, rate, or extent of antigen processing and presentation of polysaccharide antigen via MHC class II.